D-arabinitol dehydrogenase (NADP+) activity [GO:0033709] (molecular function) Also known as: D-arabinitol dehydrogenase 1 activity, D-arabinitol:NADP+ dehydrogenase activity, NADP+-dependent D-arabinitol dehydrogenase activity, ARD1p, D-arabinitol dehydrogenase, D-ribulose forming (NADP+) activity, D-arabinitol dehydrogenase, D-xylulose forming (NADP+) activity Relationships: is a type of oxidoreductase activity, acting on the CH-OH group of donors, NAD or NADP as acceptor [GO:0016616] Definition: Catalysis of the reaction: D-arabinitol + NADP+ = D-ribulose + NADPH + H+. Can also produce D-ribulose. Sources: EC:1.1.1.287